{
  "gene_symbol": "GFRA1",
  "gene": "UniProtKB:P56159",
  "term_id": "GO:0038023",
  "gene_name": "GDNF family receptor alpha-1",
  "term_label": "signaling receptor activity"
}